{
  "gene_name": "Aquaporin-3",
  "gene_symbol": "AQP3",
  "gene": "UniProtKB:Q92482",
  "term_label": "water channel activity",
  "term_id": "GO:0015250"
}